renal system development [GO:0072001] (BP) Relationships: is a type of GO:0048731 Definition: The process whose specific outcome is the progression of the renal system over time, from its formation to the mature structure. The renal system maintains fluid balance and contributes to electrolyte balance, acid/base balance, and disposal of nitrogenous waste products. In humans, the renal system comprises a pair of kidneys, a pair of ureters, urinary bladder, urethra, sphincter muscle and associated blood vessels. References: PMID:6996269 Sources: GOC:mtg_kidney_jan10, GOC:yaf Also known as: urinary system development, urinary tract development